{
  "term_label": "cytoplasm",
  "gene_symbol": "NUDT3",
  "gene": "UniProtKB:O95989",
  "term_id": "GO:0005737",
  "gene_name": "Diphosphoinositol polyphosphate phosphohydrolase 1"
}